{
  "gene_symbol": "TMPRSS5",
  "term_id": "GO:0016485",
  "gene_name": "Transmembrane protease serine 5",
  "gene": "UniProtKB:Q9H3S3",
  "term_label": "protein processing"
}